stachyose metabolic process [GO:0033531] (biological process) Also known as: stachyose metabolism Subtypes: stachyose biosynthetic process [GO:0033532] Relationships: is a type of oligosaccharide metabolic process [GO:0009311] Definition: The chemical reactions and pathways involving stachyose, the tetrasaccharide beta-D-fructofuranosyl alpha-D-galactopyranosyl-(1->6)-alpha-D-galactopyranosyl-(1->6)-alpha-D-glucopyranoside. Sources: GOC:mah